{
  "gene_name": "MTOR-associated protein MEAK7",
  "term_id": "GO:0006979",
  "gene": "UniProtKB:Q6P9B6",
  "term_label": "response to oxidative stress",
  "gene_symbol": "MEAK7"
}